L-idonate catabolic process [GO:0046183] (biological process) Sources: GOC:curators Relationships: is a type of GO:0016052; is a type of aldonic acid catabolic process [GO:0046176] Definition: The chemical reactions and pathways resulting in the breakdown of L-idonate, the anion of idonic acid, an aldonic acid derived from L-idose, an aldohexose which is epimeric with D-glucose. Also known as: L-idonate breakdown, L-idonate catabolism, L-idonate degradation